calcitriol biosynthetic process from calciol [GO:0036378] (biological process) Relationships: is a type of vitamin D biosynthetic process [GO:0042368]; is a type of polyol biosynthetic process [GO:0046173]; is a type of vitamin D3 metabolic process [GO:0070640] References: PMID:17426122, PMID:20511049 Sources: GOC:BHF, GOC:rl Also known as: 1alpha,25(OH)2D3 biosynthesis, 1alpha,25-dihydroxycholecalciferol biosynthesis, 1alpha,25-dihydroxyvitamin D3 biosynthesis, calcitriol biosynthesis from calciol, vitamin D3 activation Definition: Conversion of vitamin D3 from its largely inactive form (calciol, also called cholecalciferol) into a hormonally active form (calcitriol). Conversion requires 25-hydroxylation of calciol in the liver to form calcidiol, and subsequent 1,alpha-hydroxylation of calcidiol in the kidney to form calcitriol.